positive regulation of DNA replication [GO:0045740] (biological process) Sources: GOC:go_curators Definition: Any process that activates or increases the frequency, rate or extent of DNA replication. Also known as: up regulation of DNA replication, up-regulation of DNA replication, upregulation of DNA replication, activation of DNA replication, stimulation of DNA replication Subtypes: positive regulation of DNA-templated DNA replication [GO:2000105] Relationships: is a type of regulation of DNA replication [GO:0006275]; is a type of positive regulation of DNA metabolic process [GO:0051054]; positively regulates GO:0006260